Noc complex [GO:0030689] (cellular component) References: PMID:12446671 Definition: Any of several heterodimers containing one or two Noc proteins, associated with preribosomal complexes; involved in ribosome biogenesis. Relationships: is a type of nuclear protein-containing complex [GO:0140513] Subtypes: Noc1p-Noc2p complex [GO:0030690], GO:0030691, Noc4p-Nop14p complex [GO:0030692] Note: Noc complexes exhibit a dynamic intranuclear location; consider also annotating to 'nucleolus ; GO:0005730' and/or 'nucleoplasm ; GO:0005654'. Note that the definition uses Saccharomyces gene product names because this complex has only been described in Saccharomyces cerevisiae and no other names have yet arisen; the term nevertheless can be used for analogous complexes in other eukaryotes, and the definition can be changed if better wording is found.